{
  "gene_symbol": "OR7A17",
  "gene": "UniProtKB:O14581",
  "term_id": "GO:0007165",
  "term_label": "signal transduction",
  "gene_name": "Olfactory receptor 7A17"
}